{
  "gene_name": "Putative HLA class I histocompatibility antigen, alpha chain H",
  "term_id": "GO:0006955",
  "gene": "UniProtKB:P01893",
  "gene_symbol": "HLA-H",
  "term_label": "immune response"
}